{
  "gene": "UniProtKB:Q86WV1",
  "gene_symbol": "SKAP1",
  "term_id": "GO:0005737",
  "gene_name": "Src kinase-associated phosphoprotein 1",
  "term_label": "cytoplasm"
}